G protein-coupled neurotensin receptor activity [GO:0016492] (molecular function) Relationships: is a type of GO:0008188 Also known as: G protein coupled neurotensin receptor activity, G-protein coupled neurotensin receptor activity, neurotensin receptor activity, G protein coupled, neurotensin receptor activity, G-protein coupled References: PMID:10390649 Definition: Combining with the tridecapeptide neurotensin to initiate a G-protein mediated change in cell activity. A G-protein is a signal transduction molecule that alternates between an inactive GDP-bound and an active GTP-bound state.